{
  "gene_name": "Neuronal acetylcholine receptor subunit beta-4",
  "term_label": "plasma membrane",
  "term_id": "GO:0005886",
  "gene_symbol": "CHRNB4",
  "gene": "UniProtKB:P30926"
}